{
  "gene_name": "Olfactory receptor 2M2",
  "term_label": "detection of chemical stimulus involved in sensory perception of smell",
  "gene": "UniProtKB:Q96R28",
  "term_id": "GO:0050911",
  "gene_symbol": "OR2M2"
}